{
  "term_id": "GO:0005737",
  "gene": "UniProtKB:Q9BXJ9",
  "gene_name": "N-alpha-acetyltransferase 15, NatA auxiliary subunit",
  "term_label": "cytoplasm",
  "gene_symbol": "NAA15"
}